pseudopodium [GO:0031143] (cellular component) Also known as: pseudopod, pseudopodial protrusion, axopodium, lobopodium, reticulopodium Sources: ISBN:0198506732 Relationships: is a type of GO:0120025 Definition: A temporary protrusion or retractile process of a cell, associated with flowing movements of the protoplasm, and serving for locomotion and feeding.